reservosome lumen [GO:0106124] (cellular component) Relationships: is a type of cellular anatomical structure [GO:0110165]; is part of GO:0106123 Definition: The volume enclosed by the membranes of a reservosome. References: PMID:12204365, PMID:15521631, PMID:18452191, PMID:19288526, PMID:21818313, PMID:22425988 Sources: GOC:ach